RNA polymerase I complex [GO:0005736] (cellular component) Relationships: is a type of GO:0000428; is a type of GO:0140513; BFO_0000050 nucleolus [GO:0005730] Sources: GOC:krc, GOC:mtg_sensu Also known as: DNA-directed RNA polymerase I complex, DNA-directed RNA polymerase I activity Definition: RNA polymerase I, one of three nuclear DNA-directed RNA polymerases found in all eukaryotes, is a multisubunit complex; typically it produces rRNAs. Two large subunits comprise the most conserved portion including the catalytic site and share similarity with other eukaryotic and bacterial multisubunit RNA polymerases. The remainder of the complex is composed of smaller subunits (generally ten or more), some of which are also found in RNA polymerase III and others of which are also found in RNA polymerases II and III. Although the core is competent to mediate ribonucleic acid synthesis, it requires additional factors to select the appropriate template.